{
  "term_id": "GO:0061630",
  "gene_name": "E3 ubiquitin-protein ligase TM129",
  "gene": "UniProtKB:A0AVI4",
  "gene_symbol": "TMEM129",
  "term_label": "ubiquitin protein ligase activity"
}